{
  "term_label": "Unknown molecular function",
  "gene_symbol": "FMN1",
  "gene": "UniProtKB:Q68DA7",
  "gene_name": "Formin-1",
  "term_id": "UNKNOWN:0001"
}